{
  "gene_name": "Signal-regulatory protein beta-1",
  "term_id": "GO:0050870",
  "gene": "UniProtKB:O00241",
  "gene_symbol": "SIRPB1",
  "term_label": "positive regulation of T cell activation"
}